{
  "gene": "UniProtKB:Q8N9T2",
  "gene_symbol": "NKAPP1",
  "term_label": "Unknown molecular function",
  "term_id": "UNKNOWN:0001",
  "gene_name": "Putative uncharacterized protein CXorf42"
}